{
  "term_id": "UNKNOWN:0002",
  "gene": "UniProtKB:O00559",
  "gene_symbol": "EBAG9",
  "term_label": "Unknown biological process",
  "gene_name": "Receptor-binding cancer antigen expressed on SiSo cells"
}